{
  "gene": "UniProtKB:Q8TAU3",
  "gene_name": "Zinc finger protein 417",
  "gene_symbol": "ZNF417",
  "term_id": "GO:0006357",
  "term_label": "regulation of transcription by RNA polymerase II"
}